{
  "term_label": "immunoglobulin complex",
  "gene_name": "Immunoglobulin kappa variable 4-1",
  "gene_symbol": "IGKV4-1",
  "gene": "UniProtKB:P06312",
  "term_id": "GO:0019814"
}